{
  "gene_symbol": "PDCD6IP",
  "gene": "UniProtKB:Q8WUM4",
  "gene_name": "Programmed cell death 6-interacting protein",
  "term_id": "GO:0000281",
  "term_label": "mitotic cytokinesis"
}